{
  "gene": "UniProtKB:Q9UGM1",
  "term_label": "transmembrane transporter complex",
  "term_id": "GO:1902495",
  "gene_name": "Neuronal acetylcholine receptor subunit alpha-9",
  "gene_symbol": "CHRNA9"
}